{
  "term_label": "nucleus",
  "term_id": "GO:0005634",
  "gene": "UniProtKB:Q8WVV9",
  "gene_symbol": "HNRNPLL",
  "gene_name": "Heterogeneous nuclear ribonucleoprotein L-like"
}